{
  "gene": "UniProtKB:Q9NZN8",
  "term_label": "nuclear-transcribed mRNA poly(A) tail shortening",
  "gene_symbol": "CNOT2",
  "term_id": "GO:0000289",
  "gene_name": "CCR4-NOT transcription complex subunit 2"
}